metanephric intraglomerular mesangial cell proliferation [GO:0072263] (biological process) Sources: GOC:mtg_kidney_jan10 Definition: The multiplication or reproduction of intraglomerular glomerular mesangium cells in the metanephros by cell division, resulting in the expansion of their population. Intraglomerular mesangial cells are specialized pericytes located among the glomerular capillaries within a renal corpuscle of a kidney. They are required for filtration, structural support and phagocytosis. Relationships: is a type of intraglomerular mesangial cell proliferation [GO:0072123]; is a type of metanephric glomerular mesangial cell proliferation involved in metanephros development [GO:0072262]